{
  "term_label": "cytoplasm",
  "gene_symbol": "GRK7",
  "term_id": "GO:0005737",
  "gene_name": "Rhodopsin kinase GRK7",
  "gene": "UniProtKB:Q8WTQ7"
}